{
  "gene": "UniProtKB:P39748",
  "gene_symbol": "FEN1",
  "term_id": "GO:0008409",
  "term_label": "5'-3' exonuclease activity",
  "gene_name": "Flap endonuclease 1"
}